{
  "term_id": "GO:0050852",
  "gene": "UniProtKB:Q7KYR7",
  "gene_name": "Butyrophilin subfamily 2 member A1",
  "gene_symbol": "BTN2A1",
  "term_label": "T cell receptor signaling pathway"
}